{
  "term_label": "Unknown biological process",
  "term_id": "UNKNOWN:0002",
  "gene": "UniProtKB:A6NMA1",
  "gene_name": "Putative uncharacterized protein TRPC5OS",
  "gene_symbol": "TRPC5OS"
}